{
  "gene_symbol": "GGT3P",
  "gene": "UniProtKB:A6NGU5",
  "gene_name": "Putative glutathione hydrolase 3 proenzyme",
  "term_id": "GO:0006751",
  "term_label": "glutathione catabolic process"
}